{
  "gene_name": "Pleckstrin homology-like domain family A member 2",
  "gene": "UniProtKB:Q53GA4",
  "term_id": "UNKNOWN:0003",
  "gene_symbol": "PHLDA2",
  "term_label": "Unknown cellular component"
}